{
  "term_id": "GO:0008532",
  "gene": "UniProtKB:Q9Y2A9",
  "term_label": "N-acetyllactosaminide beta-1,3-N-acetylglucosaminyltransferase activity",
  "gene_name": "N-acetyllactosaminide beta-1,3-N-acetylglucosaminyltransferase 3",
  "gene_symbol": "B3GNT3"
}